{
  "gene": "UniProtKB:P01825",
  "term_label": "Unknown cellular component",
  "gene_name": "Immunoglobulin heavy variable 4-59",
  "gene_symbol": "IGHV4-59",
  "term_id": "UNKNOWN:0003"
}